regulation of seedling development [GO:1900140] (biological process) Sources: GOC:TermGenie Subtypes: regulation of seed germination [GO:0010029] Relationships: is a type of regulation of post-embryonic development [GO:0048580]; regulates GO:0090351 Definition: Any process that modulates the frequency, rate or extent of seedling development.